{
  "gene_name": "DENN domain-containing protein 5A",
  "gene": "UniProtKB:Q6IQ26",
  "term_id": "GO:0042147",
  "gene_symbol": "DENND5A",
  "term_label": "retrograde transport, endosome to Golgi"
}